{
  "gene": "UniProtKB:O75152",
  "term_label": "poly(A)+ mRNA export from nucleus",
  "gene_name": "Zinc finger CCCH domain-containing protein 11A",
  "gene_symbol": "ZC3H11A",
  "term_id": "GO:0016973"
}